positive regulation of tRNA processing [GO:2000237] (biological process) Also known as: positive regulation of tRNA maturation Subtypes: positive regulation of tRNA methylation [GO:0110004] Sources: GOC:mah Relationships: is a type of positive regulation of gene expression [GO:0010628]; is a type of positive regulation of tRNA metabolic process [GO:1903328]; is a type of regulation of tRNA processing [GO:2000235]; positively regulates tRNA processing [GO:0008033] Definition: Any process that activates or increases the frequency, rate or extent of tRNA processing.